{
  "term_label": "cysteine-type endopeptidase activity",
  "gene": "UniProtKB:Q96DT6",
  "gene_symbol": "ATG4C",
  "term_id": "GO:0004197",
  "gene_name": "Cysteine protease ATG4C"
}